{
  "term_label": "endosome",
  "term_id": "GO:0005768",
  "gene_symbol": "RAB40AL",
  "gene_name": "Ras-related protein Rab-40A-like",
  "gene": "UniProtKB:P0C0E4"
}